diterpenoid metabolic process [GO:0016101] (biological process) Subtypes: retinoid metabolic process [GO:0001523], GO:0009685, diterpenoid biosynthetic process [GO:0016102], diterpenoid catabolic process [GO:0016103], phytol metabolic process [GO:0033306] Sources: ISBN:0198547684 Definition: The chemical reactions and pathways involving diterpenoid compounds, terpenoids with four isoprene units. Also known as: diterpenoid metabolism, diterpene metabolic process, diterpene metabolism Relationships: is a type of terpenoid metabolic process [GO:0006721]